{
  "gene_symbol": "USP1",
  "term_label": "nucleus",
  "term_id": "GO:0005634",
  "gene": "UniProtKB:O94782",
  "gene_name": "Ubiquitin carboxyl-terminal hydrolase 1"
}